{
  "gene_name": "Sorting nexin-18",
  "gene_symbol": "SNX18",
  "term_label": "cleavage furrow formation",
  "gene": "UniProtKB:Q96RF0",
  "term_id": "GO:0036089"
}